extracellular transport [GO:0006858] (BP) Sources: GOC:go_curators Definition: The transport of substances that occurs outside cells. Subtypes: epithelial cilium movement involved in extracellular fluid movement [GO:0003351], extracellular amino acid transport [GO:0006860] Relationships: is a type of GO:0006810; occurs in extracellular region [GO:0005576]